{
  "term_label": "brush border",
  "gene_name": "Sodium-dependent phosphate transport protein 2B",
  "term_id": "GO:0005903",
  "gene": "UniProtKB:O95436",
  "gene_symbol": "SLC34A2"
}